{
  "gene_symbol": "EXOSC10",
  "term_id": "GO:0071036",
  "gene": "UniProtKB:Q01780",
  "gene_name": "Exosome component 10",
  "term_label": "nuclear polyadenylation-dependent snoRNA catabolic process"
}